regulatory ncRNA-mediated heterochromatin formation [GO:0031048] (biological process) References: PMID:19239886, PMID:21420348 Regulation: regulated by GO:0010964; negatively regulated by negative regulation of regulatory ncRNA-mediated heterochromatin formation [GO:0060906] Definition: A heterochromatin formation-based gene silencing process mediated by a regulatory non-coding RNA molecule that occur before the beginning of trancription. Relationships: is a type of regulatory ncRNA-mediated gene silencing [GO:0031047]; is_a GO:0031507 Subtypes: GO:0140966, siRNA-mediated heterochromatin formation [GO:0141194] Also known as: RNA-mediated TGS, pre-transcriptional gene silencing by RNA, RNA interference-like chromatin silencing, RNA-dependent heterochromatin formation, RNA-mediated chromatin silencing, RNA-mediated transcriptional silencing, RNAi-directed chromatin silencing, RNAi-like chromatin silencing, ncRNA-mediated heterochromatin formation, heterochromatin assembly by small RNA, pre-transcriptional gene silencing by small non-coding RNA, small RNA-mediated heterochromatic silencing, small RNA-mediated heterochromatin formation, small ncRNA-mediated heterochromatin formation, small non-coding RNA-dependent heterochromatin formation, RNA-mediated heterochromatin formation, chromatin silencing by small RNA, heterochromatin assembly involved in chromatin silencing by small RNA, heterochromatin formation involved in chromatin silencing by small RNA